{
  "gene": "UniProtKB:P13378",
  "gene_name": "Homeobox protein Hox-D8",
  "term_label": "RNA polymerase II transcription regulatory region sequence-specific DNA binding",
  "term_id": "GO:0000977",
  "gene_symbol": "HOXD8"
}